G protein-coupled histamine receptor binding [GO:0031806] (MF) Definition: Binding to a G protein-coupled (metabotropic) histamine receptor. Relationships: is_a G protein-coupled receptor binding [GO:0001664] References: PMID:12679144 Sources: GOC:mah, GOC:nln Subtypes: GO:0031807, H2 histamine receptor binding [GO:0031808], H3 histamine receptor binding [GO:0031809], H4 histamine receptor binding [GO:0031810] Also known as: G-protein coupled histamine receptor binding, metabotropic histamine receptor binding, metabotropic histamine receptor ligand